alpha2-adrenergic receptor activity [GO:0004938] (molecular function) Definition: Combining with epinephrine or norepinephrine to initiate a change in cell activity via activation of a G protein, with pharmacological characteristics of alpha2-adrenergic receptors; the activity involves transmitting the signal to the Gi alpha subunit of a heterotrimeric G protein. Sources: GOC:cb, GOC:mah, IUPHAR_GPCR:1274 Also known as: alpha2 adrenoceptor Relationships: is a type of GO:0004936